{
  "gene": "UniProtKB:Q96I13",
  "gene_symbol": "ABHD8",
  "term_label": "phosphatidic acid biosynthetic process",
  "gene_name": "Protein ABHD8",
  "term_id": "GO:0006654"
}